{
  "gene_name": "Endothelin-1",
  "gene_symbol": "EDN1",
  "term_id": "GO:0005179",
  "gene": "UniProtKB:P05305",
  "term_label": "hormone activity"
}